open rectifier potassium channel activity [GO:0005252] (molecular function) Relationships: is_a voltage-gated potassium channel activity [GO:0005249] Definition: Enables the transmembrane transfer of a potassium ion by an open rectifier voltage-gated channel. An open rectifier current-voltage relationship is one in which the direction of rectification depends on the external potassium ion concentration. References: PMID:8917578 Sources: GOC:mah